{
  "gene_name": "Conserved oligomeric Golgi complex subunit 4",
  "term_id": "UNKNOWN:0001",
  "gene": "UniProtKB:Q9H9E3",
  "gene_symbol": "COG4",
  "term_label": "Unknown molecular function"
}